translation activator activity [GO:0008494] (molecular function) Definition: Any of a group of soluble proteins functioning in the activation of ribosome-mediated translation of mRNA into a polypeptide. Sources: GOC:ai Relationships: is a type of translation regulator activity [GO:0045182]; is part of positive regulation of translation [GO:0045727]